{
  "gene_symbol": "HLA-B",
  "gene_name": "HLA class I histocompatibility antigen, B alpha chain",
  "term_label": "antigen processing and presentation of endogenous peptide antigen via MHC class I via ER pathway, TAP-independent",
  "gene": "UniProtKB:P01889",
  "term_id": "GO:0002486"
}